{
  "term_id": "GO:0005615",
  "gene_symbol": "C8A",
  "term_label": "extracellular space",
  "gene": "UniProtKB:P07357",
  "gene_name": "Complement component C8 alpha chain"
}